{
  "gene_name": "Unconventional myosin-X",
  "gene_symbol": "MYO10",
  "term_id": "GO:0051489",
  "term_label": "regulation of filopodium assembly",
  "gene": "UniProtKB:Q9HD67"
}